{
  "gene": "UniProtKB:Q13163",
  "gene_name": "Dual specificity mitogen-activated protein kinase kinase 5",
  "term_id": "GO:0004708",
  "term_label": "MAP kinase kinase activity",
  "gene_symbol": "MAP2K5"
}